{
  "gene": "UniProtKB:Q969S9",
  "term_label": "mitochondrial translation",
  "gene_symbol": "GFM2",
  "gene_name": "Ribosome-releasing factor 2, mitochondrial",
  "term_id": "GO:0032543"
}